{
  "term_label": "cell surface",
  "gene_name": "Glypican-2",
  "gene_symbol": "GPC2",
  "term_id": "GO:0009986",
  "gene": "UniProtKB:Q8N158"
}